{
  "gene_name": "p53 apoptosis effector related to PMP-22",
  "gene": "UniProtKB:Q96FX8",
  "gene_symbol": "PERP",
  "term_id": "GO:0098609",
  "term_label": "cell-cell adhesion"
}